{
  "term_id": "GO:0021987",
  "gene_symbol": "BTBD3",
  "gene": "UniProtKB:Q9Y2F9",
  "term_label": "cerebral cortex development",
  "gene_name": "BTB_POZ domain-containing protein 3"
}